regulation of apoptosis involved in tissue homeostasis [GO:0060785] (biological process) Relationships: is a type of regulation of apoptotic process [GO:0042981]; is part of homeostasis of number of cells within a tissue [GO:0048873] Sources: GOC:dph Definition: Any process that modulates the occurrence or rate of cell death by apoptosis that results in the maintenance of the steady-state number of cells within a tissue.